{
  "term_id": "GO:0015193",
  "gene": "UniProtKB:Q495M3",
  "gene_symbol": "SLC36A2",
  "term_label": "L-proline transmembrane transporter activity",
  "gene_name": "Proton-coupled amino acid transporter 2"
}